5-(carboxyamino)imidazole ribonucleotide mutase activity [GO:0034023] (molecular function) Also known as: 5-carboxyamino-1-(5-phospho-D-ribosyl)imidazole carboxymutase activity, N5-CAIR mutase activity, N5-carboxyaminoimidazole ribonucleotide mutase activity, PurE, class I PurE Sources: EC:5.4.99.18 Relationships: is a type of intramolecular transferase activity [GO:0016866] Definition: Catalysis of the reaction: 5-carboxyamino-1-(5-phospho-D-ribosyl)imidazole = 5-amino-1-(5-phospho-D-ribosyl)imidazole-4-carboxylate.